{
  "gene_name": "Ankyrin repeat and SOCS box protein 17",
  "gene": "UniProtKB:Q8WXJ9",
  "gene_symbol": "ASB17",
  "term_label": "Unknown biological process",
  "term_id": "UNKNOWN:0002"
}